{
  "gene_name": "Growth hormone-releasing hormone receptor",
  "term_label": "growth hormone-releasing hormone receptor activity",
  "gene": "UniProtKB:Q02643",
  "gene_symbol": "GHRHR",
  "term_id": "GO:0016520"
}